{
  "gene": "UniProtKB:O95475",
  "term_label": "eye development",
  "gene_name": "Homeobox protein SIX6",
  "term_id": "GO:0001654",
  "gene_symbol": "SIX6"
}